{
  "gene_name": "Craniofacial development protein 1",
  "gene_symbol": "CFDP1",
  "gene": "UniProtKB:Q9UEE9",
  "term_id": "GO:0006338",
  "term_label": "chromatin remodeling"
}